auxin influx transmembrane transporter activity [GO:0010328] (molecular function) Definition: Enables the transfer of auxin, from one side of a membrane to the other, into a cell. Also known as: auxin influx facilitator References: PMID:16839804 Relationships: is a type of auxin transmembrane transporter activity [GO:0080161]; is part of GO:0060919